{
  "term_id": "UNKNOWN:0001",
  "gene": "UniProtKB:O43837",
  "gene_symbol": "IDH3B",
  "term_label": "Unknown molecular function",
  "gene_name": "Isocitrate dehydrogenase [NAD] subunit beta, mitochondrial"
}